mRNA stabilization [GO:0048255] (biological process) Subtypes: GO:0070934, 3'-UTR-mediated mRNA stabilization [GO:0070935] Sources: GOC:jid Relationships: is a type of GO:0043488; is a type of RNA stabilization [GO:0043489]; is a type of GO:1902373 Definition: Prevention of degradation of mRNA molecules. In the absence of compensating changes in other processes, the slowing of mRNA degradation can result in an overall increase in the population of active mRNA molecules.